{
  "term_id": "GO:0070373",
  "gene": "UniProtKB:P51452",
  "gene_symbol": "DUSP3",
  "term_label": "negative regulation of ERK1 and ERK2 cascade",
  "gene_name": "Dual specificity protein phosphatase 3"
}